{
  "gene_symbol": "KRTAP9-4",
  "term_label": "Unknown cellular component",
  "term_id": "UNKNOWN:0003",
  "gene": "UniProtKB:Q9BYQ2",
  "gene_name": "Keratin-associated protein 9-4"
}